{
  "gene": "UniProtKB:Q8N1G2",
  "term_id": "GO:0006370",
  "term_label": "7-methylguanosine mRNA capping",
  "gene_name": "Cap-specific mRNA (nucleoside-2'-O-)-methyltransferase 1",
  "gene_symbol": "CMTR1"
}